{
  "term_label": "nucleus",
  "term_id": "GO:0005634",
  "gene_symbol": "UBN2",
  "gene": "UniProtKB:Q6ZU65",
  "gene_name": "Ubinuclein-2"
}